{
  "gene": "UniProtKB:P00540",
  "term_id": "GO:0005737",
  "gene_symbol": "MOS",
  "term_label": "cytoplasm",
  "gene_name": "Proto-oncogene serine_threonine-protein kinase mos"
}